{
  "gene_symbol": "NSMAF",
  "term_label": "tumor necrosis factor-mediated signaling pathway",
  "gene": "UniProtKB:Q92636",
  "gene_name": "Protein FAN",
  "term_id": "GO:0033209"
}